bacterial-type flagellum organization [GO:0044781] (biological process) Definition: A process that is carried out at the cellular level which results in the assembly, arrangement of constituent parts, or disassembly of a bacterial-type flagellum, a motor complex composed of an extracellular helical protein filament coupled to a rotary motor embedded in the cell envelope which functions in cell motility. Sources: GOC:jl Subtypes: bacterial-type flagellum assembly [GO:0044780] Relationships: is a type of GO:0006996; is a type of cell projection organization [GO:0030030]